{
  "gene_name": "Cyclic AMP-dependent transcription factor ATF-2",
  "gene_symbol": "ATF2",
  "gene": "UniProtKB:P15336",
  "term_label": "Unknown cellular component",
  "term_id": "UNKNOWN:0003"
}